{
  "term_id": "GO:0045047",
  "gene_symbol": "SRPRB",
  "term_label": "protein targeting to ER",
  "gene": "UniProtKB:Q9Y5M8",
  "gene_name": "Signal recognition particle receptor subunit beta"
}